{
  "gene_symbol": "CYP17A1",
  "gene": "UniProtKB:P05093",
  "term_label": "steroid 17-alpha-monooxygenase activity",
  "term_id": "GO:0004508",
  "gene_name": "Steroid 17-alpha-hydroxylase_17,20 lyase"
}